3,4-didehydroretinal binding [GO:0046876] (molecular function) Relationships: is a type of GO:0005501 Sources: GOC:ai, ISBN:0198506732 Definition: Binding to 3,4-didehydroretinal, a form of retinal that plays a role in the visual process in freshwater fish and some amphibians analogous to that of all-trans retinal in other vertebrates. 3,4-didehydro-11-cis-retinal combines with an opsin to form cyanopsin (cone) or porphyropsin (rod). Also known as: UV-sensitive opsin, blue-sensitive opsin, green-sensitive opsin, long-wave-sensitive opsin, opsin, red-sensitive opsin, short-wave-sensitive opsin, violet-sensitive opsin